{
  "gene": "UniProtKB:P18848",
  "gene_name": "Cyclic AMP-dependent transcription factor ATF-4",
  "gene_symbol": "ATF4",
  "term_label": "regulation of transcription by RNA polymerase II",
  "term_id": "GO:0006357"
}